{
  "term_label": "glutamine N-acyltransferase activity",
  "gene": "UniProtKB:A0A0U1RQE8",
  "gene_symbol": "GLYATL1B",
  "term_id": "GO:0047946",
  "gene_name": "Putative glycine N-acyltransferase-like protein 1B"
}